{
  "term_label": "heparin binding",
  "gene": "UniProtKB:Q99435",
  "gene_name": "Protein kinase C-binding protein NELL2",
  "gene_symbol": "NELL2",
  "term_id": "GO:0008201"
}